{
  "gene_name": "BTB_POZ domain-containing protein 6",
  "gene_symbol": "BTBD6",
  "term_label": "Unknown molecular function",
  "term_id": "UNKNOWN:0001",
  "gene": "UniProtKB:Q96KE9"
}